{
  "term_id": "UNKNOWN:0003",
  "gene_name": "Zinc finger protein 710",
  "gene_symbol": "ZNF710",
  "gene": "UniProtKB:Q8N1W2",
  "term_label": "Unknown cellular component"
}